regulation of dopamine biosynthetic process [GO:1903179] (biological process) Definition: Any process that modulates the frequency, rate or extent of dopamine biosynthetic process. Subtypes: GO:1903180, positive regulation of dopamine biosynthetic process [GO:1903181] Also known as: regulation of dopamine anabolism, regulation of dopamine biosynthesis, regulation of dopamine formation, regulation of dopamine synthesis Relationships: is a type of GO:0009889; is a type of regulation of dopamine metabolic process [GO:0042053]; regulates dopamine biosynthetic process [GO:0042416] Sources: GOC:PARL, GOC:TermGenie, GOC:bf, GO_REF:0000058